folic acid transport [GO:0015884] (biological process) Sources: GOC:ai Also known as: folate transport, vitamin B9 transport, vitamin M transport Relationships: is a type of GO:0006835; is a type of amide transport [GO:0042886]; is a type of vitamin transport [GO:0051180]; is a type of GO:0072337 Subtypes: GO:0098838 Definition: The directed movement of folic acid (pteroylglutamic acid) into, out of or within a cell, or between cells, by means of some agent such as a transporter or pore. Folic acid is widely distributed as a member of the vitamin B complex and is essential for the synthesis of purine and pyrimidines.